{
  "term_id": "UNKNOWN:0001",
  "gene_symbol": "LRRC45",
  "gene": "UniProtKB:Q96CN5",
  "term_label": "Unknown molecular function",
  "gene_name": "Leucine-rich repeat-containing protein 45"
}